ribonuclease III activity [GO:0004525] (molecular function) Definition: Catalysis of the endonucleolytic cleavage of RNA with 5'-phosphomonoesters and 3'-OH termini; makes two staggered cuts in both strands of dsRNA, leaving a 3' overhang of 2 nt. Relationships: is a type of RNA endonuclease activity producing 5'-phosphomonoesters, hydrolytic mechanism [GO:0016891]; is a type of double-stranded RNA-specific ribonuclease activity [GO:0032296] References: PMID:11157775, PMID:15242644 Also known as: pre-mRNA 3'-end processing endonuclease, RNase III activity, ribonuclease 3 activity